{
  "term_id": "GO:0004897",
  "gene": "UniProtKB:P26992",
  "gene_symbol": "CNTFR",
  "gene_name": "Ciliary neurotrophic factor receptor subunit alpha",
  "term_label": "ciliary neurotrophic factor receptor activity"
}